negative regulation of methane biosynthetic process from 3-(methylthio)propionic acid [GO:1900334] (biological process) Sources: GOC:TermGenie, GOC:mengo_curators Definition: Any process that stops, prevents or reduces the frequency, rate or extent of methane biosynthetic process from 3-(methylthio)propionic acid. Relationships: is a type of negative regulation of fatty acid metabolic process [GO:0045922]; is a type of regulation of methane biosynthetic process from 3-(methylthio)propionic acid [GO:1900333]; is a type of GO:1901578; is a type of GO:1901856; negatively regulates GO:2001132 Also known as: down regulation of methane biosynthetic process from 3-(methylthio)propionic acid, down-regulation of methane biosynthetic process from 3-(methylthio)propionic acid, downregulation of methane biosynthetic process from 3-(methylthio)propionic acid, inhibition of methane biosynthetic process from 3-(methylthio)propionic acid